{
  "term_label": "nucleus",
  "gene": "UniProtKB:Q13526",
  "gene_symbol": "PIN1",
  "term_id": "GO:0005634",
  "gene_name": "Peptidyl-prolyl cis-trans isomerase NIMA-interacting 1"
}